{
  "gene_symbol": "VTI1B",
  "gene": "UniProtKB:Q9UEU0",
  "gene_name": "Vesicle transport through interaction with t-SNAREs homolog 1B",
  "term_id": "GO:0016236",
  "term_label": "macroautophagy"
}